{
  "gene_name": "Sodium-coupled monocarboxylate transporter 1",
  "gene": "UniProtKB:Q8N695",
  "term_id": "GO:0015730",
  "term_label": "propanoate transmembrane transport",
  "gene_symbol": "SLC5A8"
}